negative regulation of forward locomotion [GO:1905849] (biological process) Relationships: is a type of negative regulation of locomotion [GO:0040013]; is a type of regulation of forward locomotion [GO:0043059]; negatively regulates forward locomotion [GO:0043056] Definition: Any process that stops, prevents or reduces the frequency, rate or extent of forward locomotion. Also known as: down regulation of forward locomotion, down-regulation of forward locomotion, downregulation of forward locomotion, inhibition of forward locomotion References: PMID:11717360 Sources: GOC:TermGenie, GO_REF:0000058